{
  "gene_symbol": "KCNG2",
  "term_id": "GO:0071805",
  "gene_name": "Potassium voltage-gated channel subfamily G member 2",
  "term_label": "potassium ion transmembrane transport",
  "gene": "UniProtKB:Q9UJ96"
}